{
  "term_id": "UNKNOWN:0003",
  "gene_symbol": "NNT",
  "gene_name": "NAD(P) transhydrogenase, mitochondrial",
  "gene": "UniProtKB:Q13423",
  "term_label": "Unknown cellular component"
}